{
  "term_label": "nucleus",
  "gene": "UniProtKB:O75496",
  "gene_symbol": "GMNN",
  "gene_name": "Geminin",
  "term_id": "GO:0005634"
}